{
  "term_label": "negative regulation of Ras protein signal transduction",
  "gene_name": "Protein sprouty homolog 3",
  "term_id": "GO:0046580",
  "gene": "UniProtKB:O43610",
  "gene_symbol": "SPRY3"
}